Dsc E3 ubiquitin ligase complex [GO:0044695] (cellular component) Relationships: is a type of ubiquitin ligase complex [GO:0000151]; is a type of membrane protein complex [GO:0098796]; is part of organelle membrane [GO:0031090] Definition: An E3 ubiquitin ligase complex localized to the ER and Golgi membrane. In fission yeast comprises Dsc1, 2, 3 and 4. Involved in the processes of fission yeast sre1 (human SREBP) transcriptional activator proteolytic cleavage, the multivesicular body (MVB) pathway, and a post-endoplasmic reticulum pathway for protein catabolism. References: PMID:21504829 Sources: GOC:mah, GOC:vw